{
  "gene_name": "Probable carboxypeptidase X1",
  "gene": "UniProtKB:Q96SM3",
  "gene_symbol": "CPXM1",
  "term_label": "extracellular space",
  "term_id": "GO:0005615"
}